inhibin binding [GO:0034711] (molecular function) Definition: Binding to an inhibin monomer, any of the polypeptides that combine to form activin and inhibin dimers. Sources: GOC:BHF, GOC:mah Also known as: inhibin monomer binding, inhibin alpha binding, inhibin beta-A binding, inhibin beta-B binding Relationships: is a type of protein binding [GO:0005515]